negative regulation of renal water transport [GO:2001152] (biological process) Relationships: is a type of negative regulation of transport [GO:0051051]; is_a negative regulation of multicellular organismal process [GO:0051241]; is a type of regulation of renal water transport [GO:2001151]; negatively regulates GO:0003097 Definition: Any process that stops, prevents or reduces the frequency, rate or extent of renal water transport. Sources: GOC:obol